{
  "gene_symbol": "ANKRD36C",
  "term_id": "UNKNOWN:0003",
  "gene_name": "Ankyrin repeat domain-containing protein 36C",
  "term_label": "Unknown cellular component",
  "gene": "UniProtKB:Q5JPF3"
}